{
  "term_label": "adenylate cyclase-inhibiting dopamine receptor signaling pathway",
  "term_id": "GO:0007195",
  "gene_name": "D(2) dopamine receptor",
  "gene": "UniProtKB:P14416",
  "gene_symbol": "DRD2"
}